establishment of planar polarity involved in neural tube closure [GO:0090177] (biological process) Relationships: is a type of establishment of planar polarity of embryonic epithelium [GO:0042249]; is a type of embryonic morphogenesis [GO:0048598]; is part of neural tube closure [GO:0001843] Sources: GOC:ascb_2009, GOC:dph, GOC:tb Definition: Coordinated organization of groups of cells in the plane of an epithelium that contributes to the closure of the neural tube. Regulation: regulated by regulation of establishment of planar polarity involved in neural tube closure [GO:0090178]